{
  "gene_name": "Gamma-tubulin complex component 3",
  "gene": "UniProtKB:Q96CW5",
  "term_label": "microtubule nucleation",
  "term_id": "GO:0007020",
  "gene_symbol": "TUBGCP3"
}